{
  "gene": "UniProtKB:Q52LA3",
  "gene_name": "Protein lin-52 homolog",
  "gene_symbol": "LIN52",
  "term_id": "UNKNOWN:0003",
  "term_label": "Unknown cellular component"
}